positive regulation of B cell differentiation [GO:0045579] (biological process) Sources: GOC:go_curators Definition: Any process that activates or increases the frequency, rate or extent of B cell differentiation. Relationships: is a type of regulation of B cell differentiation [GO:0045577]; is_a positive regulation of lymphocyte differentiation [GO:0045621]; is a type of GO:0050871; positively regulates B cell differentiation [GO:0030183] Subtypes: positive regulation of B-1 B cell differentiation [GO:0001926], GO:0002900, positive regulation of central B cell anergy [GO:0002916], positive regulation of plasma cell differentiation [GO:1900100] Also known as: positive regulation of B lymphocyte differentiation, positive regulation of B-cell differentiation, positive regulation of B-lymphocyte differentiation, up regulation of B cell differentiation, up-regulation of B cell differentiation, upregulation of B cell differentiation, activation of B cell differentiation, stimulation of B cell differentiation, positive regulation of B cell development Note: Note that immunologists typically use the word 'development' to refer to cells of B or T cell lineages undergoing the process that GO describes as 'cell differentiation'.